{
  "term_label": "potassium channel activity",
  "gene_name": "Potassium channel subfamily U member 1",
  "term_id": "GO:0005267",
  "gene_symbol": "KCNU1",
  "gene": "UniProtKB:A8MYU2"
}